{
  "gene_symbol": "PITX3",
  "gene_name": "Pituitary homeobox 3",
  "term_id": "GO:0000981",
  "gene": "UniProtKB:O75364",
  "term_label": "DNA-binding transcription factor activity, RNA polymerase II-specific"
}